{
  "gene_name": "Rho-associated protein kinase 1",
  "gene": "UniProtKB:Q13464",
  "gene_symbol": "ROCK1",
  "term_label": "regulation of actin cytoskeleton organization",
  "term_id": "GO:0032956"
}